{
  "gene_symbol": "TGFBR3L",
  "term_id": "UNKNOWN:0003",
  "gene_name": "Transforming growth factor-beta receptor type 3-like protein",
  "gene": "UniProtKB:H3BV60",
  "term_label": "Unknown cellular component"
}